UDP-N-acetylmuramoylalanyl-D-glutamate-2,6-diaminopimelate ligase activity [GO:0008765] (molecular function) Definition: Catalysis of the reaction: meso-2,6-diaminopimelate + ATP + UDP-N-acetylmuramoyl-L-alanyl-D-glutamate = ADP + 2 H+ + phosphate + UDP-N-acetylmuramoyl-L-alanyl-D-gamma-glutamyl-meso-2,6-diaminoheptanedioate. Also known as: MurE synthetase activity, UDP-N-acetylmuramoyl-L-alanyl-D-glutamate:(L)-meso-2,6-diaminoheptanedioate gamma-ligase (ADP-forming), UDP-N-acetylmuramoyl-L-alanyl-D-glutamate:meso-2,6-diamino-heptanedioate ligase (ADP-forming) activity, UDP-N-acetylmuramoyl-L-alanyl-D-glutamyl-meso-2,6-diaminopimelate synthetase activity, UDP-N-acetylmuramyl-tripeptide synthetase activity Relationships: is a type of acid-amino acid ligase activity [GO:0016881] Sources: EC:6.3.2.13, RHEA:23676